regulation of vitamin A metabolic process [GO:1901738] (biological process) Definition: Any process that modulates the frequency, rate or extent of vitamin A metabolic process. Relationships: is a type of regulation of isoprenoid metabolic process [GO:0019747]; regulates vitamin A metabolic process [GO:0006776] References: PMID:18093975 Sources: GOC:TermGenie Also known as: regulation of vitamin A metabolism